{
  "term_id": "GO:0000151",
  "term_label": "ubiquitin ligase complex",
  "gene_symbol": "ARIH1",
  "gene": "UniProtKB:Q9Y4X5",
  "gene_name": "E3 ubiquitin-protein ligase ARIH1"
}